{
  "term_id": "GO:0007409",
  "gene_symbol": "SLITRK6",
  "term_label": "axonogenesis",
  "gene_name": "SLIT and NTRK-like protein 6",
  "gene": "UniProtKB:Q9H5Y7"
}